4-hydroxy-2-oxovalerate aldolase activity [GO:0008701] (molecular function) Definition: Catalysis of the reaction: 4-hydroxy-2-oxopentanoate = acetaldehyde + pyruvate. Sources: EC:4.1.3.39, RHEA:22624 Also known as: 4-hydroxy-2-ketovalerate aldolase activity, 4-hydroxy-2-oxopentanoate pyruvate-lyase (acetaldehyde-forming) activity, 4-hydroxy-2-oxopentanoate pyruvate-lyase activity, 4-hydroxy-2-oxovalerate pyruvate-lyase activity, DmpG, HOA Relationships: is a type of oxo-acid-lyase activity [GO:0016833]